{
  "gene_symbol": "IL11RA",
  "gene": "UniProtKB:Q14626",
  "term_label": "cytokine-mediated signaling pathway",
  "gene_name": "Interleukin-11 receptor subunit alpha",
  "term_id": "GO:0019221"
}